chylomicron assembly [GO:0034378] (biological process) Relationships: is a type of plasma lipoprotein particle assembly [GO:0034377] Sources: GOC:BHF, GOC:mah Definition: The non-covalent aggregation and arrangement of proteins and lipids in the intestine to form a chylomicron.